{
  "term_label": "cell surface receptor signaling pathway",
  "gene_name": "Interleukin-1 receptor type 2",
  "term_id": "GO:0007166",
  "gene": "UniProtKB:P27930",
  "gene_symbol": "IL1R2"
}